N-acetylmannosamine catabolic process [GO:0006053] (biological process) Also known as: N-acetylmannosamine breakdown, N-acetylmannosamine catabolism, N-acetylmannosamine degradation Sources: GOC:ai, ISBN:0198506732 Relationships: is a type of N-acetylmannosamine metabolic process [GO:0006051]; is_a mannosamine catabolic process [GO:0046346] Definition: The chemical reactions and pathways resulting in the breakdown of N-acetylmannosamine, the acetylated derivative of mannosamine, 2-amino-2-deoxymannose.